{
  "gene": "UniProtKB:P59045",
  "term_label": "regulation of inflammatory response",
  "term_id": "GO:0050727",
  "gene_name": "NACHT, LRR and PYD domains-containing protein 11",
  "gene_symbol": "NLRP11"
}